{
  "term_id": "GO:0005886",
  "gene_name": "SH2B adapter protein 2",
  "term_label": "plasma membrane",
  "gene_symbol": "SH2B2",
  "gene": "UniProtKB:O14492"
}